COPI-coated inter-Golgi transport vesicle [GO:0030143] (cellular component) Relationships: is a type of GO:0030133; is a type of COPI-coated vesicle [GO:0030137] Also known as: inter-Golgi transport constitutive secretory pathway transport vesicle Definition: A vesicle that mediates transport of cargo within the Golgi complex (for example, between cisternae of the Golgi stack). Sources: GOC:mah